hexose oxidase activity [GO:0047979] (molecular function) Definition: Catalysis of the reaction: hexose + O2 = aldono-1,5-lactone + H202. Sources: EC:1.1.3.5 Also known as: D-hexose:oxygen 1-oxidoreductase activity Relationships: is a type of oxidoreductase activity, acting on the CH-OH group of donors, oxygen as acceptor [GO:0016899] Subtypes: beta-D-glucose oxidase activity [GO:0046562]